{
  "term_id": "GO:0030041",
  "term_label": "actin filament polymerization",
  "gene": "UniProtKB:Q27J81",
  "gene_name": "Inverted formin-2",
  "gene_symbol": "INF2"
}